{
  "term_label": "GTPase activity",
  "gene": "UniProtKB:Q05193",
  "gene_name": "Dynamin-1",
  "gene_symbol": "DNM1",
  "term_id": "GO:0003924"
}